{
  "gene_name": "C5a anaphylatoxin chemotactic receptor 1",
  "gene": "UniProtKB:P21730",
  "term_id": "GO:0002430",
  "term_label": "complement receptor mediated signaling pathway",
  "gene_symbol": "C5AR1"
}